negative regulation of cytokinesis, actomyosin contractile ring assembly [GO:2000432] (biological process) Relationships: is a type of negative regulation of cytokinesis [GO:0032466]; is a type of negative regulation of cytoskeleton organization [GO:0051494]; is a type of regulation of cytokinesis, actomyosin contractile ring assembly [GO:2000431]; negatively regulates actomyosin contractile ring assembly [GO:0000915] Also known as: negative regulation of contractile ring assembly Sources: GOC:obol Definition: Any process that stops, prevents or reduces the frequency, rate or extent of cytokinesis, actomyosin contractile ring assembly. Subtypes: GO:1903500